{
  "term_label": "pH-gated sodium channel activity",
  "gene_symbol": "ASIC2",
  "term_id": "GO:0160125",
  "gene": "UniProtKB:Q16515",
  "gene_name": "Acid-sensing ion channel 2"
}